{
  "term_label": "Cul2-RING ubiquitin ligase complex",
  "term_id": "GO:0031462",
  "gene_symbol": "PRAMEF27",
  "gene": "UniProtKB:A3QJZ7",
  "gene_name": "PRAME family member 27"
}